{
  "term_label": "cellular response to cadmium ion",
  "term_id": "GO:0071276",
  "gene_name": "Metallothionein-1F",
  "gene": "UniProtKB:P04733",
  "gene_symbol": "MT1F"
}